cysteine synthase complex [GO:0009333] (CC) Definition: Cysteine synthase is a multienzyme complex made up, in E. coli, of the heteromeric hexamer serine acetyltransferase and the homodimer O-acetylserine (thiol)-lyase A. Relationships: is a type of GO:1990234; is part of cytoplasm [GO:0005737] References: PMID:10993149